{
  "gene_name": "Putative uncharacterized protein encoded by FER1L6-AS2",
  "gene": "UniProtKB:Q96M78",
  "term_id": "UNKNOWN:0002",
  "term_label": "Unknown biological process",
  "gene_symbol": "FER1L6-AS2"
}